{
  "gene_symbol": "PSEN1",
  "term_label": "calcium ion homeostasis",
  "gene": "UniProtKB:P49768",
  "gene_name": "Presenilin-1",
  "term_id": "GO:0055074"
}